{
  "gene_name": "Myosin regulatory light chain 12A",
  "gene": "UniProtKB:P19105",
  "term_id": "GO:0016460",
  "gene_symbol": "MYL12A",
  "term_label": "myosin II complex"
}